{
  "gene_name": "TLR4 interactor with leucine rich repeats",
  "term_label": "regulation of cytokine production involved in immune response",
  "gene_symbol": "TRIL",
  "term_id": "GO:0002718",
  "gene": "UniProtKB:Q7L0X0"
}